{
  "term_label": "Unknown molecular function",
  "gene_name": "Oncoprotein-induced transcript 3 protein",
  "gene_symbol": "OIT3",
  "term_id": "UNKNOWN:0001",
  "gene": "UniProtKB:Q8WWZ8"
}